{
  "gene_symbol": "MBNL2",
  "term_id": "GO:0043484",
  "term_label": "regulation of RNA splicing",
  "gene": "UniProtKB:Q5VZF2",
  "gene_name": "Muscleblind-like protein 2"
}